{
  "term_label": "Unknown biological process",
  "gene": "UniProtKB:Q9UND3",
  "term_id": "UNKNOWN:0002",
  "gene_name": "Nuclear pore complex-interacting protein family member A1",
  "gene_symbol": "NPIPA1"
}